tyrosine phosphorylation of STAT protein [GO:0007260] (biological process) Also known as: tyrosine phosphorylation of Stat1 protein, tyrosine phosphorylation of Stat2 protein, tyrosine phosphorylation of Stat3 protein, tyrosine phosphorylation of Stat4 protein, tyrosine phosphorylation of Stat5 protein, tyrosine phosphorylation of Stat6 protein, tyrosine phosphorylation of Stat7 protein Relationships: is_a peptidyl-tyrosine phosphorylation [GO:0018108]; is part of cell surface receptor signaling pathway via JAK-STAT [GO:0007259] References: PMID:10918594 Sources: GOC:jl Definition: The process of introducing a phosphate group to a tyrosine residue of a STAT (Signal Transducer and Activator of Transcription) protein. Regulation: regulated by GO:0042509; positively regulated by positive regulation of tyrosine phosphorylation of STAT protein [GO:0042531]; negatively regulated by negative regulation of tyrosine phosphorylation of STAT protein [GO:0042532]